{
  "term_label": "extracellular space",
  "gene_name": "Proactivator polypeptide-like 1",
  "term_id": "GO:0005615",
  "gene": "UniProtKB:Q6NUJ1",
  "gene_symbol": "PSAPL1"
}